{
  "gene_name": "Mitogen-activated protein kinase kinase kinase 9",
  "gene_symbol": "MAP3K9",
  "gene": "UniProtKB:P80192",
  "term_id": "GO:0007165",
  "term_label": "signal transduction"
}